{
  "gene": "UniProtKB:Q12791",
  "gene_name": "Calcium-activated potassium channel subunit alpha-1",
  "term_label": "large conductance calcium-activated potassium channel activity",
  "gene_symbol": "KCNMA1",
  "term_id": "GO:0060072"
}